{
  "gene": "UniProtKB:P36543",
  "gene_symbol": "ATP6V1E1",
  "term_id": "GO:0046961",
  "term_label": "proton-transporting ATPase activity, rotational mechanism",
  "gene_name": "V-type proton ATPase subunit E 1"
}